{
  "term_id": "GO:0000981",
  "gene_name": "Zinc finger protein 404",
  "gene": "UniProtKB:Q494X3",
  "term_label": "DNA-binding transcription factor activity, RNA polymerase II-specific",
  "gene_symbol": "ZNF404"
}